{
  "gene": "UniProtKB:O43670",
  "gene_name": "BUB3-interacting and GLEBS motif-containing protein ZNF207",
  "term_label": "microtubule binding",
  "term_id": "GO:0008017",
  "gene_symbol": "ZNF207"
}